{
  "gene_name": "AP-1 complex subunit gamma-1",
  "gene": "UniProtKB:O43747",
  "gene_symbol": "AP1G1",
  "term_id": "GO:0035615",
  "term_label": "clathrin adaptor activity"
}